{
  "gene_name": "Uncharacterized protein",
  "term_label": "Unknown cellular component",
  "term_id": "UNKNOWN:0003",
  "gene_symbol": "A0A5F9ZHU2",
  "gene": "UniProtKB:A0A5F9ZHU2"
}